{
  "term_label": "activation of innate immune response",
  "term_id": "GO:0002218",
  "gene_name": "Caspase recruitment domain-containing protein 8",
  "gene": "UniProtKB:Q9Y2G2",
  "gene_symbol": "CARD8"
}